{
  "gene_symbol": "CEL",
  "term_label": "Unknown cellular component",
  "gene_name": "Bile salt-activated lipase",
  "term_id": "UNKNOWN:0003",
  "gene": "UniProtKB:P19835"
}